{
  "term_id": "GO:0005615",
  "term_label": "extracellular space",
  "gene": "UniProtKB:Q8TEU8",
  "gene_symbol": "WFIKKN2",
  "gene_name": "WAP, Kazal, immunoglobulin, Kunitz and NTR domain-containing protein 2"
}